{
  "gene_name": "E3 ubiquitin-protein ligase RNF114",
  "term_id": "GO:0061630",
  "term_label": "ubiquitin protein ligase activity",
  "gene_symbol": "RNF114",
  "gene": "UniProtKB:Q9Y508"
}